{
  "gene_name": "Kinesin-like protein KIF13A",
  "term_id": "GO:0016887",
  "gene": "UniProtKB:Q9H1H9",
  "gene_symbol": "KIF13A",
  "term_label": "ATP hydrolysis activity"
}